{
  "term_label": "Unknown molecular function",
  "gene_symbol": "DEFB112",
  "gene_name": "Beta-defensin 112",
  "term_id": "UNKNOWN:0001",
  "gene": "UniProtKB:Q30KQ8"
}